{
  "gene": "UniProtKB:A6NLC5",
  "term_id": "UNKNOWN:0003",
  "gene_name": "UPF0524 protein C3orf70",
  "gene_symbol": "C3orf70",
  "term_label": "Unknown cellular component"
}